Myo2p-Vac17p-Vac8p transport complex [GO:0071563] (cellular component) Relationships: is a type of GO:0032991; is part of cytoplasm [GO:0005737] Definition: A protein complex that is involved in transport of vacuoles to a newly formed daughter cell. In yeast, this complex is composed of Myo2p, Vac17p, and Vac8p. References: PMID:12594460 Sources: GOC:jp